{
  "gene_symbol": "CRIPT",
  "term_label": "microtubule binding",
  "gene_name": "Cysteine-rich PDZ-binding protein",
  "gene": "UniProtKB:Q9P021",
  "term_id": "GO:0008017"
}